{
  "gene_name": "POM121-like protein 1",
  "gene_symbol": "A0A1W2PR80",
  "gene": "UniProtKB:A0A1W2PR80",
  "term_label": "Unknown biological process",
  "term_id": "UNKNOWN:0002"
}